{
  "gene_symbol": "SEC13",
  "gene_name": "Protein SEC13 homolog",
  "term_label": "nuclear pore outer ring",
  "gene": "UniProtKB:P55735",
  "term_id": "GO:0031080"
}